{
  "term_label": "protein processing",
  "term_id": "GO:0016485",
  "gene_name": "Brain-specific serine protease 4",
  "gene": "UniProtKB:Q9GZN4",
  "gene_symbol": "PRSS22"
}